{
  "gene_symbol": "CYP39A1",
  "term_label": "Unknown cellular component",
  "gene": "UniProtKB:Q9NYL5",
  "term_id": "UNKNOWN:0003",
  "gene_name": "24-hydroxycholesterol 7-alpha-hydroxylase"
}